{
  "gene_name": "Secretogranin-3",
  "gene": "UniProtKB:Q8WXD2",
  "term_id": "GO:0033366",
  "term_label": "protein localization to secretory granule",
  "gene_symbol": "SCG3"
}